{
  "term_id": "UNKNOWN:0003",
  "gene_name": "Protein SPATA31F1",
  "gene": "UniProtKB:Q6ZU69",
  "gene_symbol": "SPATA31F1",
  "term_label": "Unknown cellular component"
}